{
  "gene_symbol": "CYB5R3",
  "gene_name": "NADH-cytochrome b5 reductase 3",
  "term_id": "GO:0071949",
  "gene": "UniProtKB:P00387",
  "term_label": "FAD binding"
}